nucleoside metabolic process [GO:0009116] (biological process) Subtypes: pyrimidine nucleoside metabolic process [GO:0006213], ribonucleoside metabolic process [GO:0009119], deoxyribonucleoside metabolic process [GO:0009120], nucleoside biosynthetic process [GO:0009163], nucleoside catabolic process [GO:0009164], purine nucleoside metabolic process [GO:0042278], GO:0070637 Also known as: nucleoside metabolism Sources: GOC:ma Relationships: is a type of GO:0055086; is a type of carbohydrate derivative metabolic process [GO:1901135] Definition: The chemical reactions and pathways involving a nucleoside, a nucleobase linked to either beta-D-ribofuranose (a ribonucleoside) or 2-deoxy-beta-D-ribofuranose, (a deoxyribonucleoside), e.g. adenosine, guanosine, inosine, cytidine, uridine and deoxyadenosine, deoxyguanosine, deoxycytidine and thymidine (= deoxythymidine). Regulation: regulated by regulation of nucleoside metabolic process [GO:0009118]; negatively regulated by GO:0045978; positively regulated by positive regulation of nucleoside metabolic process [GO:0045979]